{
  "term_label": "Unknown molecular function",
  "gene": "UniProtKB:Q5JRM2",
  "term_id": "UNKNOWN:0001",
  "gene_name": "Uncharacterized protein CXorf66",
  "gene_symbol": "CXorf66"
}